{
  "term_label": "protein kinase C binding",
  "gene": "UniProtKB:Q99435",
  "gene_symbol": "NELL2",
  "gene_name": "Protein kinase C-binding protein NELL2",
  "term_id": "GO:0005080"
}